{
  "term_id": "UNKNOWN:0003",
  "gene_symbol": "PPP1R26",
  "gene": "UniProtKB:Q5T8A7",
  "term_label": "Unknown cellular component",
  "gene_name": "Protein phosphatase 1 regulatory subunit 26"
}